{
  "term_label": "intrinsic apoptotic signaling pathway in response to DNA damage",
  "gene": "UniProtKB:P29590",
  "gene_symbol": "PML",
  "gene_name": "Protein PML",
  "term_id": "GO:0008630"
}